{
  "gene": "UniProtKB:Q8NEF3",
  "term_label": "Unknown biological process",
  "gene_symbol": "CCDC112",
  "gene_name": "Coiled-coil domain-containing protein 112",
  "term_id": "UNKNOWN:0002"
}